{
  "gene": "UniProtKB:Q01968",
  "gene_symbol": "OCRL",
  "term_id": "GO:0005737",
  "gene_name": "Inositol polyphosphate 5-phosphatase OCRL",
  "term_label": "cytoplasm"
}